{
  "term_label": "cGMP binding",
  "term_id": "GO:0030553",
  "gene_name": "Cyclic nucleotide-gated cation channel beta-3",
  "gene": "UniProtKB:Q9NQW8",
  "gene_symbol": "CNGB3"
}